{
  "term_label": "immune response",
  "gene_symbol": "TNFSF13B",
  "term_id": "GO:0006955",
  "gene": "UniProtKB:Q9Y275",
  "gene_name": "Tumor necrosis factor ligand superfamily member 13B"
}